{
  "gene_name": "WAP four-disulfide core domain protein 8",
  "term_label": "Unknown biological process",
  "gene_symbol": "WFDC8",
  "gene": "UniProtKB:Q8IUA0",
  "term_id": "UNKNOWN:0002"
}